{
  "term_id": "GO:0061709",
  "term_label": "reticulophagy",
  "gene_symbol": "ATG2B",
  "gene_name": "Autophagy-related protein 2 homolog B",
  "gene": "UniProtKB:Q96BY7"
}